{
  "gene_name": "Taste receptor type 2 member 31",
  "term_id": "GO:0016020",
  "term_label": "membrane",
  "gene": "UniProtKB:P59538",
  "gene_symbol": "TAS2R31"
}